lipid ubiquitination [GO:0120323] (BP) Relationships: is a type of lipid modification by small protein conjugation [GO:0120322] Definition: The process in which one or more ubiquitin groups are added to a lipid. References: PMID:34012115 Sources: GOC:sp